{
  "gene_name": "UDP-glucuronosyltransferase 1A3",
  "gene_symbol": "UGT1A3",
  "term_id": "GO:0016125",
  "term_label": "sterol metabolic process",
  "gene": "UniProtKB:P35503"
}